{
  "gene": "UniProtKB:Q9Y693",
  "gene_symbol": "LHFPL6",
  "gene_name": "LHFPL tetraspan subfamily member 6 protein",
  "term_id": "UNKNOWN:0002",
  "term_label": "Unknown biological process"
}